{
  "gene_name": "Dual specificity tyrosine-phosphorylation-regulated kinase 3",
  "gene": "UniProtKB:O43781",
  "gene_symbol": "DYRK3",
  "term_id": "GO:0005634",
  "term_label": "nucleus"
}